meiotic prophase II [GO:0007136] (biological process) Definition: The cell cycle phase which is the first stage of meiosis II and during which chromosomes condense and the two daughter centrioles and their asters migrate toward the poles of the cell. Note: Note that this term should not be used for direct annotation. If you are trying to make an annotation to x phase, it is likely that the correct annotation is 'regulation of x/y phase transition' or to a process which occurs during the reported phase (i.e mitotic DNA replication for mitotic S-phase). To capture the phase when a specific location or process is observed, the phase term can be used in an annotation extension (PMID:24885854) applied to a cellular component term (with the relation exists_during) or a biological process term (with the relation happens_during). Sources: GOC:mtg_cell_cycle Relationships: is_a prophase [GO:0051324]; is a type of meiosis II cell cycle phase [GO:0098765]